{
  "term_label": "cell surface receptor signaling pathway",
  "gene": "UniProtKB:Q92637",
  "gene_name": "Putative high affinity immunoglobulin gamma Fc receptor IB",
  "term_id": "GO:0007166",
  "gene_symbol": "FCGR1BP"
}